{
  "gene": "UniProtKB:Q9UJD0",
  "term_id": "GO:0098831",
  "gene_name": "Regulating synaptic membrane exocytosis protein 3",
  "term_label": "presynaptic active zone cytoplasmic component",
  "gene_symbol": "RIMS3"
}